{
  "gene_symbol": "ABCA2",
  "gene": "UniProtKB:Q9BZC7",
  "term_id": "GO:0005319",
  "term_label": "lipid transporter activity",
  "gene_name": "ATP-binding cassette sub-family A member 2"
}